{
  "term_label": "proteolysis",
  "gene": "UniProtKB:Q76LX8",
  "gene_symbol": "ADAMTS13",
  "gene_name": "A disintegrin and metalloproteinase with thrombospondin motifs 13",
  "term_id": "GO:0006508"
}